{
  "term_id": "GO:0006882",
  "gene_symbol": "MT3",
  "term_label": "intracellular zinc ion homeostasis",
  "gene_name": "Metallothionein-3",
  "gene": "UniProtKB:P25713"
}